{
  "gene": "UniProtKB:Q9HA72",
  "gene_name": "Calcium homeostasis modulator protein 2",
  "term_id": "GO:0005261",
  "term_label": "monoatomic cation channel activity",
  "gene_symbol": "CALHM2"
}